{
  "gene": "UniProtKB:P48546",
  "gene_symbol": "GIPR",
  "gene_name": "Gastric inhibitory polypeptide receptor",
  "term_id": "GO:0007188",
  "term_label": "adenylate cyclase-modulating G protein-coupled receptor signaling pathway"
}